TAT protein transport complex [GO:0033281] (CC) Also known as: TAT protein secretion complex, TAT protein translocation system complex, Twin-arginine translocation complex Relationships: is a type of plasma membrane protein complex [GO:0098797] Sources: GOC:pamgo_curators Definition: A complex of three proteins integral to the cytoplasmic membrane of bacteria and membranes of organelles derived from bacteria (chloroplasts and mitochondria) involved in membrane transport of folded proteins.